phenylalanine dehydrogenase activity [GO:0050175] (molecular function) Definition: Catalysis of the reaction: L-phenylalanine + H2O + NAD+ = phenylpyruvate + NH3 + NADH. Sources: EC:1.4.1.20, MetaCyc:PHENYLALANINE-DEHYDROGENASE-RXN Also known as: L-phenylalanine dehydrogenase activity, L-phenylalanine:NAD+ oxidoreductase (deaminating), PHD, PheDH activity Relationships: is a type of oxidoreductase activity, acting on the CH-NH2 group of donors, NAD or NADP as acceptor [GO:0016639]